inorganic anion transport [GO:0015698] (biological process) Relationships: is a type of GO:0006810 Subtypes: GO:0000316, phosphate ion transport [GO:0006817], chloride transport [GO:0006821], molybdate ion transport [GO:0015689], antimonite transmembrane transport [GO:0015699], chlorate transport [GO:0015702], GO:0015703, iodide transport [GO:0015705], nitrite transport [GO:0015707], thiosulfate transport [GO:0015709], tellurite transport [GO:0015710], GO:0015716, inorganic diphosphate transport [GO:0030505], borate transport [GO:0046713], tungstate ion transport [GO:0070614], selenate transport [GO:0080160], inorganic anion import across plasma membrane [GO:0098658], polyphosphate import into vacuole [GO:0180042], nitrate import [GO:1902025], sulfate transmembrane transport [GO:1902358], fluoride transmembrane transport [GO:1903424] Definition: The directed movement of inorganic anions into, out of or within a cell, or between cells, by means of some agent such as a transporter or pore. Inorganic anions are atoms or small molecules with a negative charge which do not contain carbon in covalent linkage. Sources: GOC:krc